clathrin- and caveolae-independent endocytosis [GO:0160294] (biological process) Definition: An endocytosis process that internalizes cargo via small, non-coated vesicles (~40-80 nm) without relying on clathrin or caveolin and can be dynamin-dependent or dynamin-independent. Relationships: is_a endocytosis [GO:0006897] References: PMID:15668298, PMID:31976201